pulmonary vein morphogenesis [GO:0060577] (BP) Also known as: pulmonary venous blood vessel morphogenesis Sources: GOC:dph Relationships: is a type of venous blood vessel morphogenesis [GO:0048845] Definition: The process in which the anatomical structure of the pulmonary venous blood vessels are generated and organized. Pulmonary veins are blood vessels that transport blood from the lungs to the heart.